sperm annulus [GO:0097227] (cellular component) Definition: The ring-like, filamentous structure located at the distal end of the midpiece of the sperm flagellum; the annulus is thought to form a diffusion barrier between the midpiece and the principal piece and serve as a stabilizing structure for tail rigidity. Relationships: is a type of cellular anatomical structure [GO:0110165]; is part of sperm flagellum [GO:0036126] Sources: GOC:cjm, MP:0009834